CCR4 chemokine receptor binding [GO:0031729] (molecular function) Also known as: CCR4 chemokine receptor ligand Sources: GOC:mah, GOC:nln Definition: Binding to a CCR4 chemokine receptor. Relationships: is a type of CCR chemokine receptor binding [GO:0048020]